sperm-egg recognition [GO:0035036] (biological process) Relationships: is a type of cell-cell recognition [GO:0009988]; is part of single fertilization [GO:0007338] Definition: The initial contact step made between the sperm plasma membrane and outer layer of the egg during fertilization. Sources: GOC:bf Subtypes: binding of sperm to zona pellucida [GO:0007339]